ceramide phosphoethanolamine biosynthetic process [GO:1905373] (biological process) Relationships: is a type of GO:0008654; is a type of sphingolipid biosynthetic process [GO:0030148] References: PMID:25667419 Sources: GOC:TermGenie, GOC:hjd, GO_REF:0000068 Also known as: ceramide phosphoethanolamine anabolism, ceramide phosphoethanolamine biosynthesis, ceramide phosphoethanolamine formation, ceramide phosphoethanolamine synthesis Definition: The chemical reactions and pathways resulting in the formation of ceramide phosphoethanolamine.